{
  "gene_name": "Epiphycan",
  "term_label": "Unknown molecular function",
  "term_id": "UNKNOWN:0001",
  "gene": "UniProtKB:Q99645",
  "gene_symbol": "EPYC"
}